{
  "term_id": "GO:0006357",
  "gene_name": "REST corepressor 3",
  "gene_symbol": "RCOR3",
  "term_label": "regulation of transcription by RNA polymerase II",
  "gene": "UniProtKB:Q9P2K3"
}